{
  "gene_name": "Aldo-keto reductase family 1 member C1",
  "gene_symbol": "AKR1C1",
  "term_id": "GO:0005829",
  "term_label": "cytosol",
  "gene": "UniProtKB:Q04828"
}